negative regulation of phosphatase activity [GO:0010923] (biological process) Relationships: is a type of regulation of phosphatase activity [GO:0010921]; is a type of negative regulation of dephosphorylation [GO:0035305]; is a type of negative regulation of hydrolase activity [GO:0051346]; negatively regulates phosphatase activity [GO:0016791] Sources: GOC:BHF, GOC:dph, GOC:tb Definition: Any process that decreases the rate or frequency of phosphatase activity. Phosphatases catalyze the hydrolysis of phosphoric monoesters, releasing inorganic phosphate. Subtypes: negative regulation of phosphatidylinositol-3,4,5-trisphosphate 5-phosphatase activity [GO:2001145]